host cell nuclear outer membrane [GO:0044202] (cellular component) Definition: The outer, i.e. cytoplasm-facing, lipid bilayer of the host nuclear envelope; continuous with the endoplasmic reticulum of the host cell and sometimes studded with ribosomes. Sources: GOC:jl Relationships: is a type of host organelle outer membrane [GO:0039661]; is a type of host cell nuclear membrane [GO:0044200]